{
  "gene": "UniProtKB:A2RRP1",
  "gene_name": "NBAS subunit of NRZ tethering complex",
  "term_id": "GO:0070939",
  "gene_symbol": "NBAS",
  "term_label": "Dsl1/NZR complex"
}